{
  "gene": "UniProtKB:P27987",
  "gene_symbol": "ITPKB",
  "gene_name": "Inositol-trisphosphate 3-kinase B",
  "term_label": "inositol hexakisphosphate kinase activity",
  "term_id": "GO:0000828"
}